{
  "gene_name": "Protein-tyrosine kinase 2-beta",
  "gene_symbol": "PTK2B",
  "term_id": "GO:0030335",
  "term_label": "positive regulation of cell migration",
  "gene": "UniProtKB:Q14289"
}